{
  "gene_symbol": "PLAT",
  "gene": "UniProtKB:P00750",
  "gene_name": "Tissue-type plasminogen activator",
  "term_id": "GO:0048008",
  "term_label": "platelet-derived growth factor receptor signaling pathway"
}